{
  "term_id": "GO:0061844",
  "term_label": "antimicrobial humoral immune response mediated by antimicrobial peptide",
  "gene_name": "Histone H2B type F-S",
  "gene_symbol": "H2BC12L",
  "gene": "UniProtKB:P57053"
}